{
  "gene": "UniProtKB:A0A286YEY9",
  "gene_symbol": "SCYGR1",
  "term_label": "Unknown molecular function",
  "gene_name": "Small cysteine and glycine repeat-containing protein 1",
  "term_id": "UNKNOWN:0001"
}